spine apparatus assembly [GO:1905355] (BP) Also known as: spine apparatus formation, dense material assembly, dense material formation Definition: The aggregation, arrangement and bonding together of a set of components to form a spine apparatus. Relationships: is a type of organelle assembly [GO:0070925] References: PMID:12928494 Sources: GOC:PARL, GOC:TermGenie, GOC:bf, GO_REF:0000079